cyclin-dependent protein serine/threonine kinase inhibitor activity [GO:0004861] (molecular function) Definition: Binds to and stops, prevents or reduces the activity of a cyclin-dependent protein serine/threonine kinase. Also known as: cyclin-dependent protein kinase inhibitor activity, cyclin dependent protein kinase inhibitor activity, CDK inhibitor, cyclin dependent kinase inhibitor, cyclin-dependent kinase inhibitor Sources: GOC:mah, GOC:pr Relationships: is a type of cyclin-dependent protein serine/threonine kinase regulator activity [GO:0016538]; is a type of protein serine/threonine kinase inhibitor activity [GO:0030291]; negatively regulates GO:0004693